{
  "term_id": "UNKNOWN:0001",
  "gene_name": "Ankyrin repeat and SOCS box protein 15",
  "gene": "UniProtKB:Q8WXK1",
  "gene_symbol": "ASB15",
  "term_label": "Unknown molecular function"
}